{
  "term_id": "GO:0005886",
  "gene": "UniProtKB:A6NM03",
  "term_label": "plasma membrane",
  "gene_name": "Olfactory receptor 2AG2",
  "gene_symbol": "OR2AG2"
}